platelet-derived growth factor beta-receptor activity [GO:0005019] (molecular function) Definition: Combining with platelet-derived growth factor isoform PDGF-BB or PDGF-AB to initiate a change in cell activity. Relationships: is a type of GO:0005017; is part of platelet-derived growth factor receptor-beta signaling pathway [GO:0035791] References: PMID:1657917 Also known as: PDGF beta-receptor activity, betaPDGF receptor activity